{
  "term_id": "UNKNOWN:0002",
  "term_label": "Unknown biological process",
  "gene": "UniProtKB:A0A494C0B9",
  "gene_symbol": "A0A494C0B9",
  "gene_name": "Uncharacterized protein"
}